{
  "gene": "UniProtKB:P04181",
  "term_id": "GO:0042802",
  "gene_name": "Ornithine aminotransferase, mitochondrial",
  "gene_symbol": "OAT",
  "term_label": "identical protein binding"
}